{
  "gene": "UniProtKB:O00139",
  "gene_name": "Kinesin-like protein KIF2A",
  "term_label": "microtubule binding",
  "gene_symbol": "KIF2A",
  "term_id": "GO:0008017"
}